{
  "gene_symbol": "CST8",
  "term_id": "GO:0005576",
  "term_label": "extracellular region",
  "gene": "UniProtKB:O60676",
  "gene_name": "Cystatin-8"
}